{
  "gene_name": "Platelet-activating factor acetylhydrolase IB subunit beta",
  "term_id": "GO:0005875",
  "gene_symbol": "PAFAH1B1",
  "term_label": "microtubule associated complex",
  "gene": "UniProtKB:P43034"
}